{
  "gene": "UniProtKB:Q1EHB4",
  "gene_symbol": "SLC5A12",
  "gene_name": "Sodium-coupled monocarboxylate transporter 2",
  "term_id": "GO:0015129",
  "term_label": "lactate transmembrane transporter activity"
}